archaeal-type flagellum-dependent cell motility [GO:0097590] (biological process) Relationships: is a type of archaeal or bacterial-type flagellum-dependent cell motility [GO:0097588] Also known as: archaeal-type flagellar cell motility Sources: GOC:cilia, GOC:krc, Wikipedia:Flagellum#Archaeal Definition: Cell motility due to the motion of one or more archaeal-type flagella. An archaeal-type flagellum (also called archaellum) is a non-membrane-bounded organelle superficially similar to a bacterial-type flagellum, but having a different molecular structure and lacking a central channel.